indolepyruvate ferredoxin oxidoreductase activity [GO:0043805] (molecular function) Definition: Catalysis of the reaction: (indol-3-yl)pyruvate + CoA + oxidized ferredoxin = S-2-(indol-3-yl)acetyl-CoA + CO2 + reduced ferredoxin. Sources: EC:1.2.7.8 Also known as: 3-(indol-3-yl)pyruvate synthase (ferredoxin) activity, 3-(indol-3-yl)pyruvate:ferredoxin oxidoreductase (decarboxylating, CoA-indole-acetylating), IOR, indolepyruvate oxidoreductase activity Relationships: is a type of GO:0016625